{
  "gene_name": "Ras-related protein Rab-15",
  "gene": "UniProtKB:P59190",
  "term_label": "exocytosis",
  "gene_symbol": "RAB15",
  "term_id": "GO:0006887"
}